{
  "term_id": "GO:0005737",
  "gene": "UniProtKB:Q9UK22",
  "gene_symbol": "FBXO2",
  "gene_name": "F-box only protein 2",
  "term_label": "cytoplasm"
}